{
  "term_label": "Unknown cellular component",
  "gene": "UniProtKB:Q8TAV5",
  "gene_name": "Uncharacterized protein KCNJ5-AS1",
  "gene_symbol": "KCNJ5-AS1",
  "term_id": "UNKNOWN:0003"
}